{
  "term_label": "protein import into nucleus",
  "gene_symbol": "NUP85",
  "gene": "UniProtKB:Q9BW27",
  "term_id": "GO:0006606",
  "gene_name": "Nuclear pore complex protein Nup85"
}